{
  "gene_symbol": "COX6B1",
  "term_label": "respiratory chain complex IV",
  "term_id": "GO:0045277",
  "gene": "UniProtKB:P14854",
  "gene_name": "Cytochrome c oxidase subunit 6B1"
}